{
  "gene": "UniProtKB:Q00LT1",
  "term_label": "opsin binding",
  "term_id": "GO:0002046",
  "gene_symbol": "PRCD",
  "gene_name": "Photoreceptor disk component PRCD"
}